{
  "gene": "UniProtKB:Q8WUY1",
  "term_label": "Unknown biological process",
  "gene_name": "Protein THEM6",
  "gene_symbol": "THEM6",
  "term_id": "UNKNOWN:0002"
}